{
  "gene_name": "Tetraspanin-1",
  "term_label": "Unknown molecular function",
  "gene_symbol": "TSPAN1",
  "term_id": "UNKNOWN:0001",
  "gene": "UniProtKB:O60635"
}